{
  "gene": "UniProtKB:Q96T76",
  "gene_name": "MMS19 nucleotide excision repair protein homolog",
  "gene_symbol": "MMS19",
  "term_id": "UNKNOWN:0001",
  "term_label": "Unknown molecular function"
}